polyphosphate kinase activity [GO:0008976] (molecular function) Definition: Catalysis of the reaction: ATP + phosphate(n) = ADP + phosphate(n+1). Also known as: polyphosphate polymerase activity, ATP-polyphosphate phosphotransferase activity, ATP:polyphosphate phosphotransferase activity, polyphosphoric acid kinase activity Sources: EC:2.7.4.1 Relationships: is a type of kinase activity [GO:0016301]; is a type of phosphotransferase activity, phosphate group as acceptor [GO:0016776]